{
  "term_id": "GO:0006357",
  "gene": "UniProtKB:Q13227",
  "gene_symbol": "GPS2",
  "term_label": "regulation of transcription by RNA polymerase II",
  "gene_name": "G protein pathway suppressor 2"
}